{
  "gene_symbol": "CCNJ",
  "gene_name": "Cyclin-J",
  "term_id": "GO:0016538",
  "term_label": "cyclin-dependent protein serine/threonine kinase regulator activity",
  "gene": "UniProtKB:Q5T5M9"
}